{
  "gene_name": "Oligodendrocyte transcription factor 1",
  "term_id": "GO:0045944",
  "term_label": "positive regulation of transcription by RNA polymerase II",
  "gene": "UniProtKB:Q8TAK6",
  "gene_symbol": "OLIG1"
}